{
  "term_id": "GO:0004993",
  "gene_name": "5-hydroxytryptamine receptor 2B",
  "term_label": "G protein-coupled serotonin receptor activity",
  "gene": "UniProtKB:P41595",
  "gene_symbol": "HTR2B"
}